{
  "term_label": "Cul3-RING ubiquitin ligase complex",
  "gene_symbol": "KLHL4",
  "gene_name": "Kelch-like protein 4",
  "term_id": "GO:0031463",
  "gene": "UniProtKB:Q9C0H6"
}